{
  "term_id": "UNKNOWN:0002",
  "gene": "UniProtKB:Q6PEV8",
  "term_label": "Unknown biological process",
  "gene_symbol": "FAM199X",
  "gene_name": "Protein FAM199X"
}